{
  "gene_symbol": "NRF1",
  "term_id": "GO:0006357",
  "gene_name": "Nuclear respiratory factor 1",
  "gene": "UniProtKB:Q16656",
  "term_label": "regulation of transcription by RNA polymerase II"
}